{
  "gene_name": "Protein BEX2",
  "gene": "UniProtKB:Q9BXY8",
  "gene_symbol": "BEX2",
  "term_label": "signaling receptor binding",
  "term_id": "GO:0005102"
}